{
  "gene_symbol": "NDUFS3",
  "gene": "UniProtKB:O75489",
  "term_id": "UNKNOWN:0001",
  "gene_name": "NADH dehydrogenase [ubiquinone] iron-sulfur protein 3, mitochondrial",
  "term_label": "Unknown molecular function"
}